{
  "gene": "UniProtKB:Q5VT79",
  "gene_name": "Annexin A8-like protein 1",
  "gene_symbol": "ANXA8L1",
  "term_label": "vesicle membrane",
  "term_id": "GO:0012506"
}